{
  "gene_name": "Glia maturation factor beta",
  "gene_symbol": "GMFB",
  "gene": "UniProtKB:P60983",
  "term_label": "negative regulation of Arp2/3 complex-mediated actin nucleation",
  "term_id": "GO:0034316"
}